micronucleus [GO:0031040] (cellular component) Sources: GOC:ns Definition: A membrane-bounded organelle of ciliated protozoan cells that contains a diploid copy of the cell's complete genome. Sections of contiguous sequence in the macronucleus are often interrupted by internal eliminated sequences (IES), and may be permuted, in micronuclei. Genic transcription is not found in micronuclei. Some ciliate species may contain multiple micronuclei per cell. Relationships: is a type of nucleus [GO:0005634]